lamellipodium assembly involved in mesendodermal cell migration [GO:0003364] (biological process) Relationships: is_a GO:0003363; is a type of cellular component assembly involved in morphogenesis [GO:0010927]; is part of cell migration involved in mesendoderm migration [GO:0090134] Sources: GOC:ascb_2009, GOC:dph, GOC:tb Definition: Formation of a lamellipodium, a thin sheetlike extension of the surface of a migrating cell that contributes to the directed self-propelled movement of a mesendodermal cell.